{
  "gene": "UniProtKB:P04629",
  "gene_symbol": "NTRK1",
  "term_label": "positive regulation of phosphatidylinositol 3-kinase/protein kinase B signal transduction",
  "term_id": "GO:0051897",
  "gene_name": "High affinity nerve growth factor receptor"
}